{
  "gene_symbol": "E2F3",
  "term_label": "regulation of transcription by RNA polymerase II",
  "term_id": "GO:0006357",
  "gene_name": "Transcription factor E2F3",
  "gene": "UniProtKB:O00716"
}